{
  "term_label": "vesicle membrane",
  "gene_name": "Putative annexin A2-like protein",
  "term_id": "GO:0012506",
  "gene_symbol": "ANXA2P2",
  "gene": "UniProtKB:A6NMY6"
}